{
  "gene": "UniProtKB:Q6ZNA4",
  "term_id": "GO:0030511",
  "term_label": "positive regulation of transforming growth factor beta receptor signaling pathway",
  "gene_symbol": "RNF111",
  "gene_name": "E3 ubiquitin-protein ligase Arkadia"
}